{
  "gene_symbol": "IL1RL1",
  "term_label": "interleukin-33 binding",
  "term_id": "GO:0002113",
  "gene": "UniProtKB:Q01638",
  "gene_name": "Interleukin-1 receptor-like 1"
}